{
  "gene": "UniProtKB:Q6UWM5",
  "gene_symbol": "GLIPR1L1",
  "term_id": "GO:0005615",
  "gene_name": "GLIPR1-like protein 1",
  "term_label": "extracellular space"
}